{
  "gene_symbol": "HOMER2",
  "term_id": "GO:0007216",
  "gene": "UniProtKB:Q9NSB8",
  "term_label": "G protein-coupled glutamate receptor signaling pathway",
  "gene_name": "Homer protein homolog 2"
}